metaphase [GO:0051323] (BP) Subtypes: mitotic metaphase [GO:0000089], meiotic metaphase II [GO:0007137] Sources: GOC:mtg_cell_cycle Note: Note that this term should not be used for direct annotation. If you are trying to make an annotation to x phase, it is likely that the correct annotation is 'regulation of x/y phase transition' or to a process which occurs during the reported phase (i.e mitotic DNA replication for mitotic S-phase). To capture the phase when a specific location or process is observed, the phase term can be used in an annotation extension (PMID:24885854) applied to a cellular component term (with the relation exists_during) or a biological process term (with the relation happens_during). Definition: The cell cycle phase, following prophase or prometaphase in higher eukaryotes, during which chromosomes become aligned on the equatorial plate of the cell. Relationships: is a type of meiotic cell cycle phase [GO:0098762]; is part of M phase [GO:0000279]